purine alkaloid metabolic process [GO:0046446] (biological process) Subtypes: purine alkaloid biosynthetic process [GO:0009711] Relationships: is a type of alkaloid metabolic process [GO:0009820]; is_a purine-containing compound metabolic process [GO:0072521] Sources: GOC:ai Also known as: purine alkaloid metabolism Definition: The chemical reactions and pathways involving purine alkaloids, compounds derived from purine and composed of an N-containing double ring structure.